{
  "term_label": "barbed-end actin filament capping",
  "gene_name": "Supervillin",
  "gene": "UniProtKB:O95425",
  "term_id": "GO:0051016",
  "gene_symbol": "SVIL"
}